{
  "gene_symbol": "PPM1B",
  "term_label": "protein serine/threonine phosphatase activity",
  "gene": "UniProtKB:O75688",
  "gene_name": "Protein phosphatase 1B",
  "term_id": "GO:0004722"
}